{
  "gene": "UniProtKB:Q16854",
  "term_label": "deoxyguanosine kinase activity",
  "gene_name": "Deoxyguanosine kinase, mitochondrial",
  "gene_symbol": "DGUOK",
  "term_id": "GO:0004138"
}